{
  "gene_symbol": "BCAR1",
  "gene_name": "Breast cancer anti-estrogen resistance protein 1",
  "term_id": "GO:0005737",
  "term_label": "cytoplasm",
  "gene": "UniProtKB:P56945"
}